symbiont-mediated evasion of host innate immune response [GO:0141043] (biological process) Relationships: is a type of symbiont-mediated evasion of host immune response [GO:0042783] Also known as: evasion of host innate immune response, evasion of host innate immune recognition Definition: A process by which a symbiont avoids recognition by host's innate immune response by altering, concealing or destroying a conserved symbiont molecule recognized by the host. The host is defined as the larger of the organisms involved in a symbiotic interaction. References: PMID:15014080, PMID:22131330, PMID:26502908, PMID:29101229 Subtypes: symbiont-mediated evasion of recognition by host pattern recognition receptor [GO:0141141], symbiont-mediated evasion of recognition by host innate immune effector [GO:0141177]